deep fiber [GO:0032123] (CC) Relationships: is a type of cellular anatomical structure [GO:0110165]; is part of cytoskeleton [GO:0005856]; is part of oral apparatus [GO:0031912] References: PMID:10503189 Also known as: deep fibre Definition: Inward projections of the cytoskeletal structures of the oral apparatus, which form a fiber that extends past the cytostome into the cytoplasm.